L-arginine transmembrane transport [GO:1903826] (biological process) Definition: The directed movement of L-arginine across a membrane. References: PMID:18357653, PMID:22822152, PMID:8195186 Sources: GOC:TermGenie, GO_REF:0000069 Also known as: L-arginine transport, arginine transport, L-arginine import, L-arginine uptake, arginine transmembrane transport Relationships: is a type of organic cation transport [GO:0015695]; is a type of L-alpha-amino acid transmembrane transport [GO:1902475]; is a type of basic amino acid transmembrane transport [GO:1990822] Subtypes: GO:0090518